{
  "term_id": "UNKNOWN:0003",
  "gene_symbol": "CCDC83",
  "gene": "UniProtKB:Q8IWF9",
  "term_label": "Unknown cellular component",
  "gene_name": "Coiled-coil domain-containing protein 83"
}